galactogen 6-beta-galactosyltransferase activity [GO:0047255] (molecular function) Relationships: is a type of UDP-galactosyltransferase activity [GO:0035250] Sources: EC:2.4.1.205, MetaCyc:2.4.1.205-RXN Definition: Catalysis of the reaction: galactogen + UDP-galactose = 1,6-beta-D-galctosylgalactogen + UDP. Also known as: 1,6-D-galactosyltransferase activity, UDP-galactose:galactogen beta-1,6-D-galactosyltransferase activity, UDPgalactose:galactogen beta-1,6-D-galactosyltransferase activity, beta-(1,6)-D-galactosyltransferase activity, galactogen 6beta-galactosyltransferase activity, uridine diphosphogalactose-galactogen galactosyltransferase activity